{
  "gene_symbol": "POM121L1P",
  "gene": "UniProtKB:Q3SYA9",
  "term_label": "Unknown cellular component",
  "gene_name": "Putative POM121-like protein 1",
  "term_id": "UNKNOWN:0003"
}